{
  "gene_name": "Guanine nucleotide-binding protein G(t) subunit alpha-3",
  "term_id": "GO:0050908",
  "gene": "UniProtKB:A8MTJ3",
  "gene_symbol": "GNAT3",
  "term_label": "detection of light stimulus involved in visual perception"
}